{
  "gene_name": "Kinesin-1 heavy chain",
  "term_id": "GO:0008574",
  "gene_symbol": "KIF5B",
  "term_label": "plus-end-directed microtubule motor activity",
  "gene": "UniProtKB:P33176"
}